{
  "term_id": "GO:0045087",
  "term_label": "innate immune response",
  "gene_name": "Defensin alpha 4",
  "gene_symbol": "DEFA4",
  "gene": "UniProtKB:P12838"
}